{
  "term_id": "GO:0006417",
  "gene_symbol": "GTDC1",
  "gene_name": "Glycosyltransferase-like domain-containing protein 1",
  "term_label": "regulation of translation",
  "gene": "UniProtKB:Q4AE62"
}